negative regulation of mitotic recombination [GO:0045950] (biological process) Subtypes: negative regulation of telomere maintenance via recombination [GO:0032208] Relationships: is a type of GO:0000019; is a type of negative regulation of DNA recombination [GO:0045910]; negatively regulates GO:0006312 Definition: Any process that inhibits or decreases the rate of DNA recombination during mitosis. Also known as: down regulation of mitotic recombination, down-regulation of mitotic recombination, downregulation of mitotic recombination, inhibition of mitotic recombination, negative regulation of recombination within rDNA repeats Sources: GOC:go_curators, GOC:hjd